{
  "gene_name": "Calmin",
  "term_label": "actin filament binding",
  "gene": "UniProtKB:Q96JQ2",
  "term_id": "GO:0051015",
  "gene_symbol": "CLMN"
}